mesonephric distal tubule development [GO:0061274] (biological process) Sources: GOC:mtg_kidney_jan10 Definition: The process whose specific outcome is the progression of the mesonephric distal tubule over time, from its formation to the mature structure. The mesonephric distal tubule is a mesonephric nephron tubule that begins at the terminal segment of the proximal tubule and ends at the mesonephric connecting tubule. Relationships: is a type of mesonephric nephron tubule development [GO:0061242]; is a type of distal tubule development [GO:0072017]